maltose transmembrane transport [GO:1904981] (biological process) Relationships: is a type of maltose transport [GO:0015768]; is a type of carbohydrate transmembrane transport [GO:0034219] References: PMID:11136464 Sources: GOC:TermGenie, GO_REF:0000069 Definition: The process in which maltose is transported across a membrane. Subtypes: GO:0106081